{
  "term_label": "Unknown molecular function",
  "gene": "UniProtKB:A0A0K0K1C4",
  "gene_symbol": "TRBV27",
  "term_id": "UNKNOWN:0001",
  "gene_name": "T cell receptor beta variable 27"
}